{
  "gene": "UniProtKB:Q5JS37",
  "term_id": "GO:0000209",
  "gene_symbol": "NHLRC3",
  "term_label": "protein polyubiquitination",
  "gene_name": "NHL repeat-containing protein 3"
}